{
  "gene": "UniProtKB:Q5VXU9",
  "gene_name": "Protein shortage in chiasmata 1 ortholog",
  "term_label": "resolution of meiotic recombination intermediates",
  "gene_symbol": "SHOC1",
  "term_id": "GO:0000712"
}